regulation of protein glutathionylation [GO:0010732] (biological process) Definition: Any process that modulates the rate, frequency, or extent of protein glutathionylation. Protein glutathionylation is the protein modification process in which a glutathione molecule is added to a protein amino acid through a disulfide linkage. Relationships: is a type of GO:0031399; regulates protein glutathionylation [GO:0010731] Subtypes: positive regulation of protein glutathionylation [GO:0010733], negative regulation of protein glutathionylation [GO:0010734] Sources: GOC:BHF, GOC:dph, GOC:rl, GOC:tb Also known as: regulation of protein amino acid glutathionylation